{
  "gene_name": "Protein FAM83G",
  "gene_symbol": "FAM83G",
  "gene": "UniProtKB:A6ND36",
  "term_label": "nucleus",
  "term_id": "GO:0005634"
}